{
  "gene_symbol": "CNGA1",
  "gene": "UniProtKB:P29973",
  "term_id": "GO:0007606",
  "term_label": "sensory perception of chemical stimulus",
  "gene_name": "cGMP-gated cation channel alpha-1"
}